{
  "term_label": "translational elongation",
  "term_id": "GO:0006414",
  "gene_name": "Putative elongation factor 1-alpha-like 3",
  "gene_symbol": "EEF1A1P5",
  "gene": "UniProtKB:Q5VTE0"
}